{
  "gene_symbol": "BTNL10P",
  "term_label": "signaling receptor binding",
  "gene": "UniProtKB:A8MVZ5",
  "gene_name": "Putative butyrophilin-like protein 10 pseudogene",
  "term_id": "GO:0005102"
}